{
  "term_label": "extracellular space",
  "gene_name": "Spexin",
  "gene_symbol": "SPX",
  "term_id": "GO:0005615",
  "gene": "UniProtKB:Q9BT56"
}